negative regulation of transcription by RNA polymerase III [GO:0016480] (biological process) Relationships: is a type of regulation of transcription by RNA polymerase III [GO:0006359]; is a type of negative regulation of DNA-templated transcription [GO:0045892]; negatively regulates transcription by RNA polymerase III [GO:0006383] Definition: Any process that stops, prevents, or reduces the frequency, rate or extent of transcription mediated by RNA polymerase III. Also known as: down regulation of transcription from RNA polymerase III promoter, down-regulation of transcription from RNA polymerase III promoter, downregulation of transcription from RNA polymerase III promoter, negative regulation of transcription from Pol III promoter, negative regulation of transcription from RNA polymerase III promoter, inhibition of transcription from RNA polymerase III promoter Sources: GOC:go_curators